{
  "term_label": "Unknown biological process",
  "gene_symbol": "CCAR1",
  "gene_name": "Cell division cycle and apoptosis regulator protein 1",
  "term_id": "UNKNOWN:0002",
  "gene": "UniProtKB:Q8IX12"
}